{
  "gene_name": "Telomere zinc finger-associated protein",
  "gene": "UniProtKB:P10074",
  "term_id": "GO:0000978",
  "term_label": "RNA polymerase II cis-regulatory region sequence-specific DNA binding",
  "gene_symbol": "ZBTB48"
}